{
  "gene_symbol": "SEPTIN12",
  "term_id": "GO:0003924",
  "gene_name": "Septin-12",
  "gene": "UniProtKB:Q8IYM1",
  "term_label": "GTPase activity"
}